{
  "term_id": "GO:0000978",
  "term_label": "RNA polymerase II cis-regulatory region sequence-specific DNA binding",
  "gene_name": "Paired mesoderm homeobox protein 1",
  "gene_symbol": "PRRX1",
  "gene": "UniProtKB:P54821"
}